{
  "term_label": "flavin adenine dinucleotide binding",
  "gene_name": "Nitric oxide synthase, inducible",
  "term_id": "GO:0050660",
  "gene_symbol": "NOS2",
  "gene": "UniProtKB:P35228"
}